serine-type carboxypeptidase activity [GO:0004185] (molecular function) Relationships: is a type of GO:0004180; is_a serine-type exopeptidase activity [GO:0070008] Sources: https://www.ebi.ac.uk/merops/about/glossary.shtml#CARBOXYPEPTIDASE Also known as: serine carboxypeptidase activity Subtypes: serine-type D-Ala-D-Ala carboxypeptidase activity [GO:0009002], peptidoglycan L,D-transpeptidase activity [GO:0071972] Definition: Catalysis of the hydrolysis of a single C-terminal amino acid residue from the C-terminus of a polypeptide chain by a catalytic mechanism that involves a catalytic triad consisting of a serine nucleophile that is activated by a proton relay involving an acidic residue (e.g. aspartate or glutamate) and a basic residue (usually histidine).